{
  "gene_symbol": "RAC3",
  "gene_name": "Ras-related C3 botulinum toxin substrate 3",
  "term_id": "GO:0005886",
  "gene": "UniProtKB:P60763",
  "term_label": "plasma membrane"
}